U2 snRNA 2'-O-methyladenosine m6 methyltransferase activity [GO:0106347] (molecular function) Definition: Catalysis of the reaction: a 2'-O-methyladenosine in U2 snRNA + S-adenosyl-L-methionine = an N6-methyl-2'-O-methyladenosine in U2 snRNA + S-adenosyl-L-homocysteine + H+. References: PMID:31913360 Sources: RHEA:62672 Relationships: is a type of GO:0106346